T-helper 1 cell lineage commitment [GO:0002296] (biological process) Definition: The process in which a CD4-positive, alpha-beta T cell becomes committed to becoming a T-helper 1 cell, a CD4-positive, alpha-beta T cell specialized to promote immunological processes often associated with resistance to intracellular bacteria, fungi, and protozoa, and pathological conditions such as arthritis. Sources: GOC:add, ISBN:0781735149 Also known as: T-helper 1 cell fate commitment, Th1 cell lineage commitment, Th1 fate commitment Relationships: is a type of T-helper cell lineage commitment [GO:0002295]; is part of T-helper 1 cell differentiation [GO:0045063]